{
  "gene_name": "Nuclear receptor subfamily 2 group C member 2",
  "gene": "UniProtKB:P49116",
  "gene_symbol": "NR2C2",
  "term_label": "Unknown cellular component",
  "term_id": "UNKNOWN:0003"
}